{
  "term_label": "reciprocal meiotic recombination",
  "gene_name": "DNA repair protein RAD51 homolog 1",
  "gene_symbol": "RAD51",
  "gene": "UniProtKB:Q06609",
  "term_id": "GO:0007131"
}